N-sulfoglucosamine sulfohydrolase activity [GO:0016250] (molecular function) Also known as: N-sulphoglucosamine sulphohydrolase activity, 2-desoxy-D-glucoside-2-sulphamate sulphohydrolase (sulphamate sulphohydrolase), N-sulfo-D-glucosamine sulfohydrolase activity, heparin sulfamidase activity, sulfoglucosamine sulfamidase activity, sulphamidase activity Definition: Catalysis of the reaction: N-sulfo-D-glucosamine + H2O = D-glucosamine + sulfate. Relationships: is a type of hydrolase activity, acting on acid sulfur-nitrogen bonds [GO:0016826] Sources: EC:3.10.1.1